{
  "term_id": "GO:0005615",
  "gene_symbol": "TPSG1",
  "gene_name": "Tryptase gamma",
  "term_label": "extracellular space",
  "gene": "UniProtKB:Q9NRR2"
}